{
  "gene_symbol": "SOD1",
  "gene": "UniProtKB:P00441",
  "term_id": "GO:0005634",
  "term_label": "nucleus",
  "gene_name": "Superoxide dismutase [Cu-Zn]"
}